{
  "gene_symbol": "OR4K13",
  "gene_name": "Olfactory receptor 4K13",
  "term_label": "Unknown cellular component",
  "gene": "UniProtKB:Q8NH42",
  "term_id": "UNKNOWN:0003"
}